{
  "gene_symbol": "C1QBP",
  "gene": "UniProtKB:Q07021",
  "term_label": "cytosolic ribosome assembly",
  "gene_name": "Complement component 1 Q subcomponent-binding protein, mitochondrial",
  "term_id": "GO:0042256"
}